prospore membrane spindle pole body attachment site [GO:0070057] (cellular component) Relationships: is a type of cellular anatomical structure [GO:0110165]; is part of prospore membrane [GO:0005628] Definition: The region of the prospore membrane to which the spindle pole body (SPB) is anchored; the prospore membrane extends from the SPB attachment site to surround the spore nucleus. Also known as: forespore membrane SPB attachment site, forespore membrane spindle pole body attachment site, prospore membrane SPB attachment site References: PMID:14702385 Sources: GOC:mah